{
  "gene_name": "5-hydroxytryptamine receptor 1E",
  "gene": "UniProtKB:P28566",
  "gene_symbol": "HTR1E",
  "term_id": "GO:0007187",
  "term_label": "G protein-coupled receptor signaling pathway, coupled to cyclic nucleotide second messenger"
}